negative regulation of platelet formation [GO:1905220] (biological process) Definition: Any process that stops, prevents or reduces the frequency, rate or extent of platelet formation. Relationships: is a type of GO:0045638; is a type of GO:1905219; negatively regulates platelet formation [GO:0030220] Also known as: down regulation of platelet extrusion, down regulation of platelet formation, down-regulation of platelet extrusion, down-regulation of platelet formation, downregulation of platelet extrusion, downregulation of platelet formation, negative regulation of platelet extrusion, inhibition of platelet extrusion, inhibition of platelet formation References: PMID:10606160 Sources: GOC:TermGenie, GO_REF:0000058